{
  "gene": "UniProtKB:Q9H2A2",
  "gene_name": "2-aminomuconic semialdehyde dehydrogenase",
  "term_id": "UNKNOWN:0003",
  "term_label": "Unknown cellular component",
  "gene_symbol": "ALDH8A1"
}